{
  "term_label": "hemoglobin complex",
  "term_id": "GO:0005833",
  "gene_name": "Hemoglobin subunit delta",
  "gene": "UniProtKB:P02042",
  "gene_symbol": "HBD"
}